metanephric DCT cell fate commitment [GO:0072242] (biological process) Relationships: is a type of DCT cell fate commitment [GO:0072146]; is part of metanephric DCT cell differentiation [GO:0072240] Definition: The process in which the developmental fate of a cell becomes restricted such that it will develop into a metanephric distal convoluted tubule cell. Sources: GOC:mtg_kidney_jan10 Also known as: metanephric distal convoluted tubule cell fate commitment